{
  "term_label": "synaptic transmission, glutamatergic",
  "term_id": "GO:0035249",
  "gene_name": "Glutamate receptor ionotropic, NMDA 3B",
  "gene": "UniProtKB:O60391",
  "gene_symbol": "GRIN3B"
}